{
  "term_id": "GO:0007052",
  "term_label": "mitotic spindle organization",
  "gene": "UniProtKB:Q14204",
  "gene_symbol": "DYNC1H1",
  "gene_name": "Cytoplasmic dynein 1 heavy chain 1"
}